{
  "gene_symbol": "PRAMEF20",
  "gene": "UniProtKB:Q5VT98",
  "term_label": "ubiquitin-like ligase-substrate adaptor activity",
  "term_id": "GO:1990756",
  "gene_name": "PRAME family member 20"
}